dicarboxylate-CoA ligase activity [GO:0047851] (molecular function) Definition: Catalysis of the reaction: ATP + an omega-dicarboxylic acid + CoASH= AMP + diphosphate + an omega-carboxyacyl-CoA. Sources: EC:6.2.1.23, MetaCyc:DICARBOXYLATE--COA-LIGASE-RXN Also known as: carboxylyl-CoA synthetase activity, omega-dicarboxylate:CoA ligase (AMP-forming) Relationships: is a type of acid-thiol ligase activity [GO:0016878]